{
  "gene_name": "Metallothionein-2",
  "gene_symbol": "MT2A",
  "term_label": "detoxification of copper ion",
  "term_id": "GO:0010273",
  "gene": "UniProtKB:P02795"
}